{
  "gene_symbol": "SLC17A7",
  "term_id": "GO:0098700",
  "term_label": "neurotransmitter loading into synaptic vesicle",
  "gene_name": "Vesicular glutamate transporter 1",
  "gene": "UniProtKB:Q9P2U7"
}